aspartate:alanine antiporter activity [GO:0070906] (MF) Also known as: aspartate-alanine antiporter activity, aspartate/alanine antiporter activity Relationships: is a type of GO:0005310; is a type of GO:0015297; is a type of C4-dicarboxylate transmembrane transporter activity [GO:0015556]; is a type of alanine transmembrane transporter activity [GO:0022858] Sources: GOC:dh Definition: Catalysis of the reaction: aspartate(out) + alanine(in) = aspartate(in) + alanine(out).